{
  "gene_symbol": "ZMYM2",
  "gene": "UniProtKB:Q9UBW7",
  "term_label": "Unknown biological process",
  "term_id": "UNKNOWN:0002",
  "gene_name": "Zinc finger MYM-type protein 2"
}